{
  "gene": "UniProtKB:Q13257",
  "term_id": "GO:0007094",
  "gene_name": "Mitotic spindle assembly checkpoint protein MAD2A",
  "gene_symbol": "MAD2L1",
  "term_label": "mitotic spindle assembly checkpoint signaling"
}